interleukin-4 receptor activity [GO:0004913] (molecular function) Definition: Combining with interleukin-4 and transmitting the signal from one side of the membrane to the other to initiate a change in cell activity. Sources: GOC:jl, GOC:signaling Also known as: IL-4 receptor activity, IL-4R Relationships: is a type of cytokine receptor activity [GO:0004896]; is part of interleukin-4-mediated signaling pathway [GO:0035771]; has part interleukin-4 binding [GO:0019979]